protein-DNA covalent cross-linking activity [GO:0160129] (molecular function) Definition: Catalysis of the cross-link between a protein and a DNA abasic site, forming a thiazolidine linkage between a DNA ring-opened abasic site and the alpha-amino and sulfhydryl substituents of cysteine residue of the protein. References: PMID:30554877, PMID:31235913 Relationships: is a type of lyase activity [GO:0016829]